{
  "gene": "UniProtKB:Q9UEW8",
  "term_label": "intracellular signal transduction",
  "gene_symbol": "STK39",
  "term_id": "GO:0035556",
  "gene_name": "STE20_SPS1-related proline-alanine-rich protein kinase"
}